{
  "gene_symbol": "ZKSCAN1",
  "gene": "UniProtKB:P17029",
  "gene_name": "Zinc finger protein with KRAB and SCAN domains 1",
  "term_id": "GO:0006357",
  "term_label": "regulation of transcription by RNA polymerase II"
}